{
  "gene_symbol": "ATP6V0A2",
  "gene": "UniProtKB:Q9Y487",
  "gene_name": "V-type proton ATPase 116 kDa subunit a 2",
  "term_id": "GO:0005886",
  "term_label": "plasma membrane"
}